{
  "gene_name": "Eukaryotic translation initiation factor 1",
  "gene": "UniProtKB:P41567",
  "term_label": "translation initiation factor activity",
  "gene_symbol": "EIF1",
  "term_id": "GO:0003743"
}